{
  "gene_symbol": "FCGR2B",
  "term_id": "GO:0009897",
  "gene": "UniProtKB:P31994",
  "gene_name": "Low affinity immunoglobulin gamma Fc region receptor II-b",
  "term_label": "external side of plasma membrane"
}